{
  "term_id": "UNKNOWN:0003",
  "gene_name": "Neutral alpha-glucosidase C",
  "gene": "UniProtKB:Q8TET4",
  "term_label": "Unknown cellular component",
  "gene_symbol": "GANC"
}